positive regulation of cell differentiation involved in phenotypic switching [GO:1905917] (BP) Definition: Any process that activates or increases the frequency, rate or extent of cell differentiation involved in phenotypic switching. Relationships: is a type of positive regulation of cell differentiation [GO:0045597]; is a type of regulation of cell differentiation involved in phenotypic switching [GO:1905915]; positively regulates cell differentiation involved in phenotypic switching [GO:0090679] Subtypes: GO:1905932 References: PMID:25089138 Sources: GOC:BHF, GOC:BHF_miRNA, GOC:TermGenie, GOC:rph, GO_REF:0000058 Also known as: up regulation of cell differentiation involved in phenotypic switching, up-regulation of cell differentiation involved in phenotypic switching, upregulation of cell differentiation involved in phenotypic switching, activation of cell differentiation involved in phenotypic switching